{
  "gene_symbol": "HES5",
  "gene_name": "Transcription factor HES-5",
  "term_id": "GO:0000981",
  "term_label": "DNA-binding transcription factor activity, RNA polymerase II-specific",
  "gene": "UniProtKB:Q5TA89"
}